{
  "gene_name": "Serine-threonine kinase receptor-associated protein",
  "term_id": "GO:0032797",
  "gene_symbol": "STRAP",
  "term_label": "SMN complex",
  "gene": "UniProtKB:Q9Y3F4"
}